{
  "term_id": "GO:0030350",
  "gene_name": "Cytoplasmic aconitate hydratase",
  "term_label": "iron-responsive element binding",
  "gene_symbol": "ACO1",
  "gene": "UniProtKB:P21399"
}